{
  "term_label": "Gemini of Cajal bodies",
  "gene_symbol": "SMN2",
  "gene": "UniProtKB:Q16637",
  "gene_name": "Survival motor neuron protein",
  "term_id": "GO:0097504"
}